{
  "term_label": "positive regulation of transcription by RNA polymerase II",
  "gene_symbol": "NR1I3",
  "gene": "UniProtKB:Q14994",
  "term_id": "GO:0045944",
  "gene_name": "Nuclear receptor subfamily 1 group I member 3"
}